germacrene-D synthase activity [GO:0052577] (molecular function) Relationships: is a type of sesquiterpene synthase activity [GO:0010334] Also known as: (2E,6E)-farnesyl-diphosphate diphosphate-lyase [(-)-germacrene-D-forming] activity Definition: Catalysis of the reaction: (2E,6E)-farnesyl diphosphate = (-)-germacrene D + diphosphate. Sources: RHEA:12016